{
  "term_id": "UNKNOWN:0001",
  "gene_name": "Inactive N-acetylated-alpha-linked acidic dipeptidase-like protein 2",
  "gene_symbol": "NAALADL2",
  "term_label": "Unknown molecular function",
  "gene": "UniProtKB:Q58DX5"
}